{
  "term_label": "positive regulation of autophagy",
  "gene_symbol": "PRKAA1",
  "term_id": "GO:0010508",
  "gene": "UniProtKB:Q13131",
  "gene_name": "5'-AMP-activated protein kinase catalytic subunit alpha-1"
}